{
  "term_id": "GO:0005743",
  "gene_name": "Cytochrome c oxidase assembly factor 3 homolog, mitochondrial",
  "term_label": "mitochondrial inner membrane",
  "gene_symbol": "COA3",
  "gene": "UniProtKB:Q9Y2R0"
}